{
  "gene_symbol": "PLEKHA3",
  "term_id": "GO:0042147",
  "gene": "UniProtKB:Q9HB20",
  "term_label": "retrograde transport, endosome to Golgi",
  "gene_name": "Pleckstrin homology domain-containing family A member 3"
}